{
  "term_id": "GO:0005886",
  "term_label": "plasma membrane",
  "gene": "UniProtKB:Q9BV40",
  "gene_name": "Vesicle-associated membrane protein 8",
  "gene_symbol": "VAMP8"
}